{
  "term_label": "immune response",
  "gene": "UniProtKB:A0JD37",
  "gene_name": "T cell receptor delta variable 3",
  "term_id": "GO:0006955",
  "gene_symbol": "TRDV3"
}